{
  "term_id": "GO:0000981",
  "gene_symbol": "ZKSCAN7",
  "term_label": "DNA-binding transcription factor activity, RNA polymerase II-specific",
  "gene_name": "Zinc finger protein with KRAB and SCAN domains 7",
  "gene": "UniProtKB:Q9P0L1"
}